9,10-epoxystearate hydroxylase activity [GO:0103004] (molecular function) Definition: Catalysis of the reaction: H+ + 9,10-epoxystearate + O2 + NADPH = 9,10-epoxy-18-hydroxystearate + H2O + NADP. Sources: GOC:pz Relationships: is a type of GO:0016709